{
  "term_label": "cyclin-dependent protein kinase holoenzyme complex",
  "gene_symbol": "CCNJ",
  "gene_name": "Cyclin-J",
  "term_id": "GO:0000307",
  "gene": "UniProtKB:Q5T5M9"
}